beta-glucogallin-tetrakisgalloylglucose O-galloyltransferase activity [GO:0047176] (molecular function) Relationships: is a type of acyltransferase activity, transferring groups other than amino-acyl groups [GO:0016747] Also known as: 1-O-galloyl-beta-D-glucose:1,2,3,6-tetrakis-O-galloyl-beta-D-glucose 4-O-galloyltransferase activity, beta-glucogallin-tetragalloylglucose 4-galloyltransferase activity, beta-glucogallin:1,2,3,6-tetra-O-galloyl-beta-D-glucose 4-O-galloyltransferase activity, beta-glucogallin:1,2,3,6-tetra-O-galloylglucose 4-O-galloyltransferase activity Sources: EC:2.3.1.143, RHEA:19109 Definition: Catalysis of the reaction: 1,2,3,6-tetrakis-O-galloyl-beta-D-glucose + 1-O-galloyl-beta-D-glucose = 1,2,3,4,6-pentakis-O-galloyl-beta-D-glucose + D-glucose.